{
  "gene": "UniProtKB:P07205",
  "gene_name": "Phosphoglycerate kinase 2",
  "gene_symbol": "PGK2",
  "term_id": "GO:0006094",
  "term_label": "gluconeogenesis"
}